negative regulation of macrophage fusion [GO:0034240] (biological process) Sources: GOC:mah Definition: Any process that stops, prevents, or decreases the frequency, rate or extent of macrophage fusion. Relationships: is a type of regulation of macrophage fusion [GO:0034239]; is a type of negative regulation of syncytium formation by plasma membrane fusion [GO:0034242]; negatively regulates macrophage fusion [GO:0034238]